iris morphogenesis [GO:0061072] (biological process) Sources: GOC:dph Relationships: is a type of anatomical structure morphogenesis [GO:0009653]; BFO_0000050 camera-type eye morphogenesis [GO:0048593] Definition: The process in which the iris is generated and organized. The iris is an anatomical structure in the eye whose opening forms the pupil. The iris is responsible for controlling the diameter and size of the pupil and the amount of light reaching the retina.